{
  "gene": "UniProtKB:Q9H425",
  "gene_name": "Uncharacterized protein C1orf198",
  "term_id": "UNKNOWN:0003",
  "gene_symbol": "C1orf198",
  "term_label": "Unknown cellular component"
}